{
  "term_id": "UNKNOWN:0003",
  "gene": "UniProtKB:Q8TA86",
  "gene_name": "Retinitis pigmentosa 9 protein",
  "term_label": "Unknown cellular component",
  "gene_symbol": "RP9"
}